{
  "term_id": "UNKNOWN:0001",
  "gene_name": "Solute carrier family 22 member 3",
  "gene_symbol": "SLC22A3",
  "gene": "UniProtKB:O75751",
  "term_label": "Unknown molecular function"
}